{
  "term_label": "Unknown molecular function",
  "gene": "UniProtKB:Q5DJT8",
  "gene_symbol": "CT45A2",
  "term_id": "UNKNOWN:0001",
  "gene_name": "Cancer_testis antigen family 45 member A2"
}